{
  "term_label": "carbohydrate binding",
  "gene_symbol": "LGALS2",
  "term_id": "GO:0030246",
  "gene": "UniProtKB:P05162",
  "gene_name": "Galectin-2"
}